G protein-coupled glucose receptor activity [GO:1990576] (molecular function) References: PMID:15667320 Also known as: G-protein coupled glucose receptor activity Relationships: is a type of G protein-coupled receptor activity [GO:0004930] Definition: Combining with an extracellular glucose molecule and transmitting the signal across the membrane by activating an associated G-protein; promotes the exchange of GDP for GTP on the alpha subunit of a heterotrimeric G-protein complex.